positive regulation of microglial cell activation [GO:1903980] (biological process) Definition: Any process that activates or increases the frequency, rate or extent of microglial cell activation. References: PMID:19100238 Sources: GOC:BHF, GOC:TermGenie, GOC:nc, GO_REF:0000058 Also known as: up regulation of microglial cell activation, up-regulation of microglial cell activation, upregulation of microglial cell activation, activation of microglial cell activation Relationships: is_a positive regulation of macrophage activation [GO:0043032]; is a type of positive regulation of neuroinflammatory response [GO:0150078]; is a type of regulation of microglial cell activation [GO:1903978]; positively regulates GO:0001774